{
  "term_id": "GO:0005737",
  "term_label": "cytoplasm",
  "gene_symbol": "CDK2AP2",
  "gene_name": "Cyclin-dependent kinase 2-associated protein 2",
  "gene": "UniProtKB:O75956"
}